{
  "term_label": "nucleus",
  "gene": "UniProtKB:Q8TAP4",
  "gene_symbol": "LMO3",
  "term_id": "GO:0005634",
  "gene_name": "LIM domain only protein 3"
}